{
  "gene_symbol": "IL15RA",
  "gene_name": "Interleukin-15 receptor subunit alpha",
  "term_label": "interleukin-15 receptor activity",
  "gene": "UniProtKB:Q13261",
  "term_id": "GO:0042010"
}